positive regulation of chondrocyte proliferation [GO:1902732] (biological process) References: PMID:23212449 Sources: GOC:TermGenie, GO_REF:0000058 Also known as: positive regulation of cartilage cell proliferation, positive regulation of chondrocyte cell proliferation, up regulation of cartilage cell proliferation, up regulation of chondrocyte cell proliferation, up regulation of chondrocyte proliferation, up-regulation of cartilage cell proliferation, up-regulation of chondrocyte cell proliferation, up-regulation of chondrocyte proliferation, upregulation of cartilage cell proliferation, upregulation of chondrocyte cell proliferation, upregulation of chondrocyte proliferation, activation of cartilage cell proliferation, activation of chondrocyte cell proliferation, activation of chondrocyte proliferation Definition: Any process that increases the frequency, rate or extent of the multiplication or reproduction of chondrocytes by cell division, resulting in the expansion of their population. A chondrocyte is a polymorphic cell that forms cartilage. Relationships: is a type of positive regulation of cell population proliferation [GO:0008284]; positively regulates chondrocyte proliferation [GO:0035988]